{
  "gene_symbol": "LINC00612",
  "term_label": "Unknown biological process",
  "term_id": "UNKNOWN:0002",
  "gene_name": "Putative uncharacterized protein encoded by LINC00612",
  "gene": "UniProtKB:Q8N6U2"
}